monocyte antigen processing and presentation [GO:0002471] (biological process) References: PMID:11200054 Sources: GOC:add Definition: The process in which a monocyte expresses antigen (peptide or lipid) on its cell surface in association with an MHC protein complex. Relationships: is a type of antigen processing and presentation [GO:0019882] Regulation: regulated by regulation of monocyte antigen processing and presentation [GO:0002613]; RO_0002212 by GO:0002614; positively regulated by positive regulation of monocyte antigen processing and presentation [GO:0002615]